{
  "term_id": "GO:0050253",
  "gene_name": "Bile salt-activated lipase",
  "gene": "UniProtKB:P19835",
  "gene_symbol": "CEL",
  "term_label": "retinyl-palmitate esterase activity"
}